{
  "gene": "UniProtKB:P01282",
  "gene_name": "VIP peptides",
  "term_label": "peptide hormone receptor binding",
  "term_id": "GO:0051428",
  "gene_symbol": "VIP"
}